{
  "gene_name": "Recoverin",
  "gene": "UniProtKB:P35243",
  "term_id": "GO:0009966",
  "gene_symbol": "RCVRN",
  "term_label": "regulation of signal transduction"
}